{
  "term_id": "GO:0007155",
  "term_label": "cell adhesion",
  "gene_name": "Sialic acid-binding Ig-like lectin 10",
  "gene_symbol": "SIGLEC10",
  "gene": "UniProtKB:Q96LC7"
}